{
  "gene_symbol": "LRRC10",
  "term_label": "cardiac muscle cell development",
  "term_id": "GO:0055013",
  "gene": "UniProtKB:Q5BKY1",
  "gene_name": "Leucine-rich repeat-containing protein 10"
}